{
  "gene_name": "EF-hand domain-containing family member B",
  "term_id": "GO:0005879",
  "gene_symbol": "EFHB",
  "term_label": "axonemal microtubule",
  "gene": "UniProtKB:Q8N7U6"
}